{
  "gene": "UniProtKB:O60861",
  "term_label": "cytoplasm",
  "term_id": "GO:0005737",
  "gene_name": "Growth arrest-specific protein 7",
  "gene_symbol": "GAS7"
}